{
  "gene": "UniProtKB:Q8NCN5",
  "gene_name": "Pyruvate dehydrogenase phosphatase regulatory subunit, mitochondrial",
  "term_label": "Unknown molecular function",
  "term_id": "UNKNOWN:0001",
  "gene_symbol": "PDPR"
}